{
  "gene": "UniProtKB:P40313",
  "term_label": "proteolysis",
  "gene_name": "Chymotrypsin-like protease CTRL-1",
  "gene_symbol": "CTRL",
  "term_id": "GO:0006508"
}